{
  "term_label": "structural constituent of chromatin",
  "term_id": "GO:0030527",
  "gene": "UniProtKB:Q7Z2G1",
  "gene_symbol": "H2BW1",
  "gene_name": "Histone H2B type W-T"
}